{
  "gene": "UniProtKB:Q6ZMM2",
  "gene_symbol": "ADAMTSL5",
  "term_id": "UNKNOWN:0002",
  "term_label": "Unknown biological process",
  "gene_name": "ADAMTS-like protein 5"
}